positive regulation of cell proliferation involved in compound eye morphogenesis [GO:2000497] (biological process) Definition: Any process that activates or increases the frequency, rate or extent of cell proliferation involved in compound eye morphogenesis. Sources: GOC:obol Relationships: is a type of positive regulation of cell population proliferation [GO:0008284]; is a type of GO:2000495; positively regulates cell proliferation involved in compound eye morphogenesis [GO:0035736]